{
  "term_id": "GO:0042796",
  "term_label": "snRNA transcription by RNA polymerase III",
  "gene_symbol": "SNAPC1",
  "gene_name": "snRNA-activating protein complex subunit 1",
  "gene": "UniProtKB:Q16533"
}